{
  "gene_symbol": "BAP1",
  "gene_name": "Ubiquitin carboxyl-terminal hydrolase BAP1",
  "gene": "UniProtKB:Q92560",
  "term_id": "GO:0031507",
  "term_label": "heterochromatin formation"
}